{
  "gene": "UniProtKB:Q15043",
  "term_id": "GO:0071578",
  "gene_name": "Metal cation symporter ZIP14",
  "gene_symbol": "SLC39A14",
  "term_label": "zinc ion import across plasma membrane"
}